maintenance of presynaptic active zone structure [GO:0048790] (biological process) Sources: GOC:curators, GOC:dph, GOC:pr Also known as: maintenance of pre-synaptic active zone structure Relationships: is a type of maintenance of synapse structure [GO:0099558]; is a type of presynaptic active zone organization [GO:1990709] Definition: A process which maintains the organization and the arrangement of proteins at the active zone to ensure the fusion and docking of vesicles and the release of neurotransmitters.